{
  "gene_name": "SEC14-like protein 1",
  "gene_symbol": "SEC14L1",
  "gene": "UniProtKB:Q92503",
  "term_label": "cytoplasm",
  "term_id": "GO:0005737"
}